{
  "term_id": "GO:0061630",
  "term_label": "ubiquitin protein ligase activity",
  "gene_symbol": "RNF115",
  "gene_name": "E3 ubiquitin-protein ligase RNF115",
  "gene": "UniProtKB:Q9Y4L5"
}